{
  "term_id": "GO:0045071",
  "gene": "UniProtKB:P13164",
  "gene_name": "Interferon-induced transmembrane protein 1",
  "gene_symbol": "IFITM1",
  "term_label": "negative regulation of viral genome replication"
}